aromatic primary alcohol metabolic process [GO:1902654] (biological process) Subtypes: aromatic primary alcohol biosynthetic process [GO:1902655] Also known as: aromatic primary alcohol metabolism Relationships: is a type of primary alcohol metabolic process [GO:0034308] References: PMID:19219878 Sources: GOC:TermGenie, GOC:mengo_curators, GO_REF:0000068 Definition: The chemical reactions and pathways involving aromatic primary alcohol.